{
  "gene_name": "Succinate dehydrogenase assembly factor 1, mitochondrial",
  "gene": "UniProtKB:A6NFY7",
  "term_id": "GO:0034553",
  "term_label": "mitochondrial respiratory chain complex II assembly",
  "gene_symbol": "SDHAF1"
}